{
  "gene_symbol": "TMEM51",
  "term_id": "UNKNOWN:0003",
  "term_label": "Unknown cellular component",
  "gene_name": "Transmembrane protein 51",
  "gene": "UniProtKB:Q9NW97"
}